{
  "gene_symbol": "DLG4",
  "term_id": "GO:0031594",
  "gene": "UniProtKB:P78352",
  "gene_name": "Disks large homolog 4",
  "term_label": "neuromuscular junction"
}